{
  "term_label": "innate immune response in mucosa",
  "gene": "UniProtKB:Q6DRA6",
  "gene_name": "Putative histone H2B type 2-D",
  "gene_symbol": "H2BC19P",
  "term_id": "GO:0002227"
}